{
  "term_id": "GO:0000398",
  "term_label": "mRNA splicing, via spliceosome",
  "gene_symbol": "RBM10",
  "gene_name": "RNA-binding protein 10",
  "gene": "UniProtKB:P98175"
}